{
  "term_label": "cytoplasm",
  "gene_name": "Crk-like protein",
  "term_id": "GO:0005737",
  "gene_symbol": "CRKL",
  "gene": "UniProtKB:P46109"
}